{
  "gene_name": "Liprin-alpha-2",
  "gene_symbol": "PPFIA2",
  "gene": "UniProtKB:O75334",
  "term_label": "Unknown molecular function",
  "term_id": "UNKNOWN:0001"
}